{
  "term_id": "GO:0005634",
  "term_label": "nucleus",
  "gene_symbol": "CCNB3",
  "gene_name": "G2_mitotic-specific cyclin-B3",
  "gene": "UniProtKB:Q8WWL7"
}